{
  "term_label": "nucleus",
  "gene_symbol": "OTUD7B",
  "gene_name": "OTU domain-containing protein 7B",
  "term_id": "GO:0005634",
  "gene": "UniProtKB:Q6GQQ9"
}